{
  "gene_symbol": "SNTG2",
  "term_id": "UNKNOWN:0001",
  "term_label": "Unknown molecular function",
  "gene": "UniProtKB:Q9NY99",
  "gene_name": "Gamma-2-syntrophin"
}